bacterial-type flagellum filament cap [GO:0009421] (cellular component) Definition: The proteinaceous structure at the distal tip of the bacterial-type flagellar filament. References: PMID:10572114, PMID:12624192 Sources: GOC:cilia, GOC:mtg_sensu Relationships: is a type of cellular anatomical structure [GO:0110165]; BFO_0000050 bacterial-type flagellum filament [GO:0009420] Also known as: flagellar filament cap, flagellin-based flagellum filament cap